{
  "gene": "UniProtKB:Q96EU6",
  "term_id": "GO:0000462",
  "gene_name": "Ribosomal RNA processing protein 36 homolog",
  "term_label": "maturation of SSU-rRNA from tricistronic rRNA transcript (SSU-rRNA, 5.8S rRNA, LSU-rRNA)",
  "gene_symbol": "RRP36"
}